XCL1 production [GO:0140779] (biological process) Relationships: is a type of cytokine production [GO:0001816] References: PMID:7973732 Note: Note that this term is in the subset of terms that should not be used for direct gene product annotation. Instead, select one of the 'regulation' children terms. Also known as: lymphotactin production Definition: The appearance of XCL1 due to biosynthesis or secretion following a cellular stimulus, resulting in an increase in its intracellular or extracellular levels.